bipolar cell growth [GO:0042815] (biological process) Sources: GOC:vw Relationships: is a type of unidimensional cell growth [GO:0009826] Also known as: bipolar growth, bipolar cell elongation, polar cell elongation Note: Bipolar cell growth refers to a change in both cell size and cell shape. For shape changes where cell size is not affected, consider instead the term 'establishment or maintenance of bipolar cell polarity resulting in cell shape ; GO:0061246' and its children. Definition: The process in which a cell irreversibly increases in size along one axis through simultaneous polarized growth from opposite ends of a cell, resulting in morphogenesis of the cell. Regulation: regulated by regulation of bipolar cell growth [GO:0051516]; negatively regulated by negative regulation of bipolar cell growth [GO:0051517]; positively regulated by positive regulation of bipolar cell growth [GO:0051518]